interleukin-11 binding [GO:0019970] (molecular function) Definition: Binding to interleukin-11. Relationships: is a type of growth factor binding [GO:0019838]; is a type of cytokine binding [GO:0019955] Sources: GOC:jl Also known as: IL-11 binding